{
  "gene": "UniProtKB:Q12965",
  "term_label": "microfilament motor activity",
  "gene_symbol": "MYO1E",
  "term_id": "GO:0000146",
  "gene_name": "Unconventional myosin-Ie"
}